{
  "term_id": "GO:0034464",
  "term_label": "BBSome",
  "gene_symbol": "BBS2",
  "gene": "UniProtKB:Q9BXC9",
  "gene_name": "Bardet-Biedl syndrome 2 protein"
}